{
  "gene_symbol": "SNTB1",
  "gene": "UniProtKB:Q13884",
  "term_id": "GO:0045202",
  "term_label": "synapse",
  "gene_name": "Beta-1-syntrophin"
}